{
  "gene_symbol": "RNF19B",
  "gene": "UniProtKB:Q6ZMZ0",
  "term_id": "GO:0044194",
  "gene_name": "E3 ubiquitin-protein ligase RNF19B",
  "term_label": "cytolytic granule"
}